{
  "term_id": "GO:0016020",
  "term_label": "membrane",
  "gene_symbol": "SLC35G4",
  "gene": "UniProtKB:P0C7Q5",
  "gene_name": "Putative solute carrier family 35 member G4"
}